{
  "term_label": "Unknown molecular function",
  "gene_name": "Immunoglobulin lambda variable 3-27",
  "term_id": "UNKNOWN:0001",
  "gene_symbol": "IGLV3-27",
  "gene": "UniProtKB:P01718"
}